{
  "term_id": "GO:0005132",
  "gene_name": "Interferon alpha-14",
  "term_label": "type I interferon receptor binding",
  "gene": "UniProtKB:P01570",
  "gene_symbol": "IFNA14"
}